{
  "gene_symbol": "TTI1",
  "term_label": "Unknown molecular function",
  "gene": "UniProtKB:O43156",
  "term_id": "UNKNOWN:0001",
  "gene_name": "TELO2-interacting protein 1 homolog"
}